{
  "gene_symbol": "PPIB",
  "term_label": "cytoplasm",
  "gene": "UniProtKB:P23284",
  "term_id": "GO:0005737",
  "gene_name": "Peptidyl-prolyl cis-trans isomerase B"
}